{
  "gene_symbol": "IMP3",
  "term_label": "Mpp10 complex",
  "gene": "UniProtKB:Q9NV31",
  "gene_name": "U3 small nucleolar ribonucleoprotein protein IMP3",
  "term_id": "GO:0034457"
}